apiose 1-reductase activity [GO:0047674] (molecular function) Sources: EC:1.1.1.114, RHEA:15301 Definition: Catalysis of the reaction: D-apiitol + NAD+ = D-apiose + H+ + NADH. Relationships: is a type of oxidoreductase activity, acting on the CH-OH group of donors, NAD or NADP as acceptor [GO:0016616] Also known as: D-apiitol reductase activity, D-apiitol:NAD+ 1-oxidoreductase activity, D-apiose reductase activity